{
  "term_id": "GO:0006995",
  "gene_symbol": "MAP1LC3B",
  "gene": "UniProtKB:Q9GZQ8",
  "term_label": "cellular response to nitrogen starvation",
  "gene_name": "Microtubule-associated proteins 1A_1B light chain 3B"
}